{
  "term_id": "GO:0005634",
  "term_label": "nucleus",
  "gene": "UniProtKB:Q6XYB7",
  "gene_symbol": "LBX2",
  "gene_name": "Transcription factor LBX2"
}